mating projection actin fusion focus [GO:1990819] (cellular component) Definition: A focus at the mating projection tip where the cell wall is degraded during conjugation with cellular fusion. Actin filaments form an aster-like structure from this location. Relationships: is a type of GO:0110165; is part of actin cytoskeleton [GO:0015629]; is part of mating projection tip [GO:0043332]; has part actin filament [GO:0005884] References: PMID:25825517 Also known as: actin fusion focus